{
  "term_label": "regulation of B cell proliferation",
  "gene_symbol": "MZB1",
  "gene_name": "Marginal zone B- and B1-cell-specific protein",
  "term_id": "GO:0030888",
  "gene": "UniProtKB:Q8WU39"
}